{
  "gene_name": "AH receptor-interacting protein",
  "term_label": "Unknown molecular function",
  "gene": "UniProtKB:O00170",
  "term_id": "UNKNOWN:0001",
  "gene_symbol": "AIP"
}